alpha-1,4-glucosidase activity [GO:0004558] (molecular function) Relationships: is a type of GO:0090599 Definition: Catalysis of the hydrolysis of terminal, non-reducing alpha-(1->4)-linked alpha-D-glucose residues with release of alpha-D-glucose. Also known as: lysosomal alpha-glucosidase activity, acid maltase activity, alpha-D-glucosidase activity, alpha-D-glucoside glucohydrolase activity, alpha-glucopyranosidase activity, alpha-glucoside hydrolase activity, glucoinvertase activity, glucosidoinvertase activity, glucosidosucrase activity, maltase-glucoamylase activity Sources: EC:3.2.1.20